fatty acid-CoA ligase activity [GO:0120515] (molecular function) Definition: Catalysis of the reaction: a fatty acid + ATP + CoA = a fatty acyl-CoA + AMP + diphosphate. Sources: RHEA:38883 Relationships: is a type of fatty acid ligase activity [GO:0015645]; is a type of CoA-ligase activity [GO:0016405] Subtypes: long-chain fatty acid-CoA ligase activity [GO:0004467], short-chain fatty acid-CoA ligase activity [GO:0031955], medium-chain fatty acid-CoA ligase activity [GO:0031956], very long-chain fatty acid-CoA ligase activity [GO:0031957]